{
  "gene": "UniProtKB:Q9Y2L9",
  "gene_name": "Leucine-rich repeat and calponin homology domain-containing protein 1",
  "term_id": "GO:0005737",
  "gene_symbol": "LRCH1",
  "term_label": "cytoplasm"
}